phragmoplast assembly [GO:0000914] (BP) Definition: The formation of a structure composed of actin, myosin, and associated proteins that will function in cytokinesis in cells that perform cytokinesis by cell plate formation. The structure usually contains antiparallel microtubules and membrane (often visible as vesicles). Also known as: phragmoplast formation Relationships: is a type of assembly of actomyosin apparatus involved in mitotic cytokinesis [GO:1902407]; BFO_0000050 cytokinesis by cell plate formation [GO:0000911] Sources: GOC:clt